{
  "term_label": "hair cycle",
  "term_id": "GO:0042633",
  "gene_name": "Keratin-associated protein 4-11",
  "gene_symbol": "KRTAP4-11",
  "gene": "UniProtKB:Q9BYQ6"
}